{
  "term_label": "Unknown molecular function",
  "gene_symbol": "DENND2D",
  "gene_name": "DENN domain-containing protein 2D",
  "term_id": "UNKNOWN:0001",
  "gene": "UniProtKB:Q9H6A0"
}